{
  "term_id": "UNKNOWN:0002",
  "term_label": "Unknown biological process",
  "gene": "UniProtKB:Q8N1A6",
  "gene_symbol": "C4orf33",
  "gene_name": "UPF0462 protein C4orf33"
}